{
  "term_id": "GO:0042393",
  "gene_name": "Condensin-2 complex subunit D3",
  "gene_symbol": "NCAPD3",
  "gene": "UniProtKB:P42695",
  "term_label": "histone binding"
}